reactive oxygen species metabolic process [GO:0072593] (biological process) Sources: GOC:mah Definition: The chemical reactions and pathways involving a reactive oxygen species, any molecules or ions formed by the incomplete one-electron reduction of oxygen. They contribute to the microbicidal activity of phagocytes, regulation of signal transduction and gene expression, and the oxidative damage to biopolymers. Also known as: ROS metabolic process, reactive oxygen species metabolism Regulation: regulated by regulation of reactive oxygen species metabolic process [GO:2000377]; negatively regulated by negative regulation of reactive oxygen species metabolic process [GO:2000378]; positively regulated by positive regulation of reactive oxygen species metabolic process [GO:2000379] Subtypes: hypochlorous acid catabolic process [GO:0002150], superoxide metabolic process [GO:0006801], hydrogen peroxide metabolic process [GO:0042743], GO:1903409 Relationships: is a type of GO:0008152